{
  "gene_symbol": "MT2A",
  "term_label": "intracellular zinc ion homeostasis",
  "gene_name": "Metallothionein-2",
  "gene": "UniProtKB:P02795",
  "term_id": "GO:0006882"
}